{
  "term_id": "GO:0055088",
  "term_label": "lipid homeostasis",
  "gene_symbol": "PNPLA3",
  "gene": "UniProtKB:Q9NST1",
  "gene_name": "1-acylglycerol-3-phosphate O-acyltransferase PNPLA3"
}